{
  "term_id": "UNKNOWN:0001",
  "gene": "UniProtKB:Q8IVU1",
  "term_label": "Unknown molecular function",
  "gene_symbol": "IGDCC3",
  "gene_name": "Immunoglobulin superfamily DCC subclass member 3"
}